{
  "gene": "UniProtKB:Q9UBY0",
  "term_id": "GO:0015386",
  "term_label": "potassium:proton antiporter activity",
  "gene_symbol": "SLC9A2",
  "gene_name": "Sodium_hydrogen exchanger 2"
}